{
  "term_id": "GO:0006357",
  "gene_symbol": "BHLHA9",
  "gene": "UniProtKB:Q7RTU4",
  "term_label": "regulation of transcription by RNA polymerase II",
  "gene_name": "Class A basic helix-loop-helix protein 9"
}